{
  "term_label": "external side of plasma membrane",
  "gene_symbol": "CXCR3",
  "term_id": "GO:0009897",
  "gene": "UniProtKB:P49682",
  "gene_name": "C-X-C chemokine receptor type 3"
}